{
  "term_id": "GO:0070653",
  "gene_name": "Apolipoprotein C-III",
  "term_label": "high-density lipoprotein particle receptor binding",
  "gene_symbol": "APOC3",
  "gene": "UniProtKB:P02656"
}